{
  "gene_name": "Vascular endothelial growth factor receptor 3",
  "term_label": "vascular endothelial growth factor receptor signaling pathway",
  "gene_symbol": "FLT4",
  "term_id": "GO:0048010",
  "gene": "UniProtKB:P35916"
}